{
  "term_id": "GO:0015937",
  "term_label": "coenzyme A biosynthetic process",
  "gene_symbol": "PANK4",
  "gene_name": "4'-phosphopantetheine phosphatase",
  "gene": "UniProtKB:Q9NVE7"
}